{
  "term_id": "GO:0034553",
  "gene_name": "Succinate dehydrogenase assembly factor 2, mitochondrial",
  "gene": "UniProtKB:Q9NX18",
  "term_label": "mitochondrial respiratory chain complex II assembly",
  "gene_symbol": "SDHAF2"
}